{
  "gene_symbol": "DTX3L",
  "gene_name": "E3 ubiquitin-protein ligase DTX3L",
  "gene": "UniProtKB:Q8TDB6",
  "term_id": "GO:0005654",
  "term_label": "nucleoplasm"
}